{
  "term_id": "UNKNOWN:0002",
  "gene_symbol": "CFAP119",
  "gene": "UniProtKB:A1A4V9",
  "gene_name": "Cilia- and flagella-associated protein 119",
  "term_label": "Unknown biological process"
}